5'-hydroxyaverantin dehydrogenase activity [GO:0140396] (molecular function) Definition: Catalyzes the reaction: (1'S,5'S)-hydroxyaverantin + NAD+ = 5'-oxoaverantin + NADH. Relationships: is a type of oxidoreductase activity, acting on the CH-OH group of donors, NAD or NADP as acceptor [GO:0016616] References: PMID:14602595 Sources: EC:1.1.1.352